{
  "term_id": "UNKNOWN:0001",
  "term_label": "Unknown molecular function",
  "gene_symbol": "CABP7",
  "gene_name": "Calcium-binding protein 7",
  "gene": "UniProtKB:Q86V35"
}